{
  "term_id": "GO:0005634",
  "gene_symbol": "FAM50B",
  "term_label": "nucleus",
  "gene": "UniProtKB:Q9Y247",
  "gene_name": "Protein FAM50B"
}